{
  "gene": "UniProtKB:Q06210",
  "term_label": "protein N-linked glycosylation",
  "term_id": "GO:0006487",
  "gene_symbol": "GFPT1",
  "gene_name": "Glutamine--fructose-6-phosphate aminotransferase [isomerizing] 1"
}